negative regulation of thyroid-stimulating hormone secretion [GO:2000613] (biological process) Also known as: negative regulation of TSH secretion, negative regulation of thyroid stimulating hormone secretion Relationships: is a type of negative regulation of peptide hormone secretion [GO:0090278]; is a type of GO:2000612; negatively regulates thyroid-stimulating hormone secretion [GO:0070460] Sources: GOC:obol Definition: Any process that stops, prevents or reduces the frequency, rate or extent of thyroid-stimulating hormone secretion.